regulation of DNA replication [GO:0006275] (biological process) Relationships: is a type of regulation of DNA metabolic process [GO:0051052]; RO_0002211 DNA replication [GO:0006260] Sources: GOC:go_curators Definition: Any process that modulates the frequency, rate or extent of DNA replication. Subtypes: negative regulation of DNA replication [GO:0008156], positive regulation of DNA replication [GO:0045740], GO:0090329